{
  "gene": "UniProtKB:A0A075B6Z0",
  "term_label": "Unknown molecular function",
  "gene_name": "T cell receptor alpha joining 22 (Fragment)",
  "gene_symbol": "TRAJ22",
  "term_id": "UNKNOWN:0001"
}